{
  "term_label": "cytosol",
  "gene_name": "Endophilin-A2",
  "term_id": "GO:0005829",
  "gene": "UniProtKB:Q99961",
  "gene_symbol": "SH3GL1"
}